{
  "gene_name": "Serine_arginine-rich splicing factor 10",
  "gene": "UniProtKB:O75494",
  "term_label": "nuclear speck",
  "term_id": "GO:0016607",
  "gene_symbol": "SRSF10"
}